{
  "gene": "UniProtKB:Q15916",
  "term_id": "GO:0001227",
  "term_label": "DNA-binding transcription repressor activity, RNA polymerase II-specific",
  "gene_name": "Zinc finger and BTB domain-containing protein 6",
  "gene_symbol": "ZBTB6"
}